{
  "gene_name": "Progonadoliberin-1",
  "gene": "UniProtKB:P01148",
  "term_label": "regulation of signaling",
  "term_id": "GO:0023051",
  "gene_symbol": "GNRH1"
}